{
  "gene_symbol": "OR5K1",
  "term_label": "Unknown cellular component",
  "term_id": "UNKNOWN:0003",
  "gene_name": "Olfactory receptor 5K1",
  "gene": "UniProtKB:Q8NHB7"
}